GTP cyclohydrolase IIa activity [GO:0043740] (molecular function) Sources: EC:3.5.4.29, RHEA:22468 Relationships: is a type of GTP cyclohydrolase activity [GO:0003933] Definition: Catalysis of the reaction: GTP + 3 H2O = 2-amino-5-formylamino-6-(5-phospho-D-ribosylamino)pyrimidin-4(3H)-one + 2 H+ + 2 phosphate. Also known as: GTP 8,9-hydrolase (phosphate-forming), GTP cyclohydrolase III activity, GTP 8,9-dihydrolase (phosphate-forming)